{
  "gene_name": "EKC_KEOPS complex subunit TP53RK",
  "term_id": "GO:0005634",
  "gene_symbol": "TP53RK",
  "term_label": "nucleus",
  "gene": "UniProtKB:Q96S44"
}